G protein-coupled receptor activity involved in regulation of postsynaptic membrane potential [GO:0099530] (molecular function) Definition: A G protein-coupled receptor activity occurring in the postsynaptic membrane that is part of a GPCR signaling pathway that positively regulates ion channel activity in the postsynaptic membrane. Relationships: is a type of GO:0004930; is part of regulation of postsynaptic membrane potential [GO:0060078]; occurs in postsynaptic membrane [GO:0045211] Subtypes: G protein-coupled neurotransmitter receptor activity involved in regulation of postsynaptic membrane potential [GO:0099579] Also known as: G-protein coupled receptor activity involved in regulation of postsynaptic membrane potential Sources: GOC:dos